{
  "gene": "UniProtKB:Q8TCJ0",
  "term_id": "GO:0005737",
  "gene_name": "F-box only protein 25",
  "gene_symbol": "FBXO25",
  "term_label": "cytoplasm"
}